peptidyl-lysine modification [GO:0018205] (biological process) Sources: GOC:go_curators Definition: The modification of peptidyl-lysine. Relationships: is a type of GO:0018193 Subtypes: GO:0008612, protein lipoylation [GO:0009249], GO:0016925, GO:0016926, peptidyl-lysine hydroxylation [GO:0017185], GO:0018022, peptidyl-lysine oxidation [GO:0018057], isopeptide cross-linking via N6-(L-isoglutamyl)-L-lysine [GO:0018153], protein-pyridoxal-5-phosphate linkage via peptidyl-N6-pyridoxal phosphate-L-lysine [GO:0018272], peptidyl-lysine acetylation [GO:0018394], peptidyl-lysine deacetylation [GO:0034983], peptidyl-lysine demalonylation [GO:0036047], peptidyl-lysine desuccinylation [GO:0036049], GO:0036528, GO:0070490, GO:0072580